{
  "gene_symbol": "CA9",
  "term_id": "GO:0005886",
  "term_label": "plasma membrane",
  "gene": "UniProtKB:Q16790",
  "gene_name": "Carbonic anhydrase 9"
}